{
  "gene_name": "Serine_threonine-protein kinase ICK",
  "term_label": "nucleus",
  "gene_symbol": "CILK1",
  "gene": "UniProtKB:Q9UPZ9",
  "term_id": "GO:0005634"
}